3-ketovalidoxylamine C-N-lyase activity [GO:0047566] (MF) Also known as: 3-ketovalidoxylamine A C-N-lyase activity, 4-nitrophenyl-3-ketovalidamine 4-nitroaniline-lyase [5-D-(5/6)-5-C-(hydroxymethyl)-2,6-dihydroxycyclohex-2-en-1-one-forming], 4-nitrophenyl-3-ketovalidamine 4-nitroaniline-lyase activity, p-nitrophenyl-3-ketovalidamine p-nitroaniline lyase activity Sources: EC:4.3.3.1, RHEA:22768 Relationships: is a type of GO:0016843 Definition: Catalysis of the reaction: 4-nitrophenyl-3-ketovalidamine = 4-nitroaniline + 5-D-(5/6)-5-C-(hydroxymethyl)-2,6-dihydroxycyclohex-2-en-1-one + H+.